{
  "gene": "UniProtKB:Q5SWW7",
  "gene_name": "Uncharacterized protein C10orf55",
  "term_id": "UNKNOWN:0002",
  "gene_symbol": "C10orf55",
  "term_label": "Unknown biological process"
}